{
  "term_label": "Unknown biological process",
  "gene_symbol": "CCDC177",
  "gene_name": "Coiled-coil domain-containing protein 177",
  "term_id": "UNKNOWN:0002",
  "gene": "UniProtKB:Q9NQR7"
}